{
  "term_label": "nucleus",
  "gene_name": "MLX-interacting protein",
  "gene_symbol": "MLXIP",
  "gene": "UniProtKB:Q9HAP2",
  "term_id": "GO:0005634"
}